{
  "term_id": "GO:0042605",
  "gene_symbol": "HLA-DQA1",
  "gene_name": "HLA class II histocompatibility antigen, DQ alpha 1 chain",
  "term_label": "peptide antigen binding",
  "gene": "UniProtKB:P01909"
}